glutaminase activity [GO:0004359] (molecular function) Relationships: is a type of hydrolase activity, acting on carbon-nitrogen (but not peptide) bonds, in linear amides [GO:0016811] Definition: Catalysis of the reaction: L-glutamine + H2O = L-glutamate + NH4+. Sources: RHEA:15889 Also known as: L-glutaminase activity, L-glutamine amidohydrolase activity, glutaminase I, glutamine aminohydrolase activity